{
  "term_label": "Unknown cellular component",
  "gene": "UniProtKB:O60232",
  "gene_name": "Protein ZNRD2",
  "gene_symbol": "ZNRD2",
  "term_id": "UNKNOWN:0003"
}